{
  "gene_symbol": "BAZ1B",
  "gene": "UniProtKB:Q9UIG0",
  "term_id": "GO:0006974",
  "gene_name": "Tyrosine-protein kinase BAZ1B",
  "term_label": "DNA damage response"
}